{
  "gene_name": "Protein ARV1",
  "term_label": "intracellular sterol transport",
  "gene": "UniProtKB:Q9H2C2",
  "gene_symbol": "ARV1",
  "term_id": "GO:0032366"
}